regulation of MAP kinase activity [GO:0043405] (biological process) Definition: Any process that modulates the frequency, rate or extent of MAP kinase activity. Sources: GOC:dph, GOC:go_curators Also known as: Regulation of MAPK activity, regulation of mitogen activated protein kinase activity, regulation of mitogen-activated protein kinase activity Relationships: is a type of GO:0071900; regulates GO:0004707 Subtypes: GO:0043406, negative regulation of MAP kinase activity [GO:0043407], regulation of JUN kinase activity [GO:0043506]